{
  "term_id": "GO:0071011",
  "gene_name": "WW domain-binding protein 4",
  "gene": "UniProtKB:O75554",
  "term_label": "precatalytic spliceosome",
  "gene_symbol": "WBP4"
}